{
  "gene_name": "TATA-binding protein-associated factor 2N",
  "term_id": "GO:0003723",
  "term_label": "RNA binding",
  "gene_symbol": "TAF15",
  "gene": "UniProtKB:Q92804"
}